{
  "term_label": "extracellular region",
  "gene_name": "Interleukin-7",
  "gene_symbol": "IL7",
  "gene": "UniProtKB:P13232",
  "term_id": "GO:0005576"
}